{
  "gene_name": "Immunoglobulin superfamily member 23",
  "term_label": "homophilic cell-cell adhesion",
  "gene_symbol": "IGSF23",
  "gene": "UniProtKB:A1L1A6",
  "term_id": "GO:0007156"
}